{
  "gene_name": "Triokinase_FMN cyclase",
  "gene": "UniProtKB:Q3LXA3",
  "gene_symbol": "TKFC",
  "term_label": "cytosol",
  "term_id": "GO:0005829"
}